{
  "term_id": "GO:0006357",
  "gene_symbol": "JADE1",
  "gene": "UniProtKB:Q6IE81",
  "term_label": "regulation of transcription by RNA polymerase II",
  "gene_name": "Protein Jade-1"
}